axonemal microtubule doublet inner junction [GO:0160113] (cellular component) Definition: The structure which joins the B10 protofilament of the B tubule to the A1 protofilament of the A tubule within an axonemal microtubule doublet. Relationships: is a type of cellular anatomical structure [GO:0110165]; is part of axonemal doublet microtubule [GO:0097545] References: PMID:29430673, PMID:37295417 Sources: GOC:krc